{
  "gene": "UniProtKB:Q8NA70",
  "gene_name": "Protein FAM47B",
  "term_id": "UNKNOWN:0001",
  "gene_symbol": "FAM47B",
  "term_label": "Unknown molecular function"
}